{
  "term_label": "axon",
  "gene_name": "Calcium and integrin-binding protein 1",
  "gene": "UniProtKB:Q99828",
  "term_id": "GO:0030424",
  "gene_symbol": "CIB1"
}